{
  "gene_symbol": "TMEM259",
  "term_label": "positive regulation of ERAD pathway",
  "term_id": "GO:1904294",
  "gene": "UniProtKB:Q4ZIN3",
  "gene_name": "Membralin"
}